{
  "term_label": "cell migration",
  "term_id": "GO:0016477",
  "gene_symbol": "CSF1R",
  "gene_name": "Macrophage colony-stimulating factor 1 receptor",
  "gene": "UniProtKB:P07333"
}